{
  "gene": "UniProtKB:A6NMY6",
  "gene_name": "Putative annexin A2-like protein",
  "term_id": "GO:0005886",
  "term_label": "plasma membrane",
  "gene_symbol": "ANXA2P2"
}